{
  "gene": "UniProtKB:Q6PIF6",
  "term_id": "GO:0000146",
  "gene_symbol": "MYO7B",
  "gene_name": "Unconventional myosin-VIIb",
  "term_label": "microfilament motor activity"
}